{
  "term_label": "Unknown cellular component",
  "gene": "UniProtKB:Q5TAG4",
  "gene_symbol": "NBPF12",
  "term_id": "UNKNOWN:0003",
  "gene_name": "Neuroblastoma breakpoint family member 12"
}